{
  "term_id": "GO:0000146",
  "term_label": "microfilament motor activity",
  "gene_symbol": "MYO9A",
  "gene_name": "Unconventional myosin-IXa",
  "gene": "UniProtKB:B2RTY4"
}